{
  "term_label": "protein phosphatase binding",
  "gene": "UniProtKB:Q9NYA4",
  "gene_name": "Myotubularin-related protein 4",
  "term_id": "GO:0019903",
  "gene_symbol": "MTMR4"
}